{
  "term_label": "Unknown biological process",
  "term_id": "UNKNOWN:0002",
  "gene": "UniProtKB:Q8N912",
  "gene_name": "Nutritionally-regulated adipose and cardiac enriched protein homolog",
  "gene_symbol": "NRAC"
}